{
  "gene": "UniProtKB:P42768",
  "term_id": "UNKNOWN:0001",
  "gene_name": "Actin nucleation-promoting factor WAS",
  "gene_symbol": "WAS",
  "term_label": "Unknown molecular function"
}